histone deacetylase activity, hydrolytic mechanism [GO:0141221] (molecular function) Also known as: histone deacetylase activity, histone deacetylase activity, NAD-independent Definition: Catalysis of the reaction: H2O + N6-acetyl-L-lysyl-[histone] = acetate + L-lysyl-[histone]. Subtypes: GO:0031078, histone H3K9 deacetylase activity, hydrolytic mechanism [GO:0032129], histone H4K16 deacetylase activity, hydrolytic mechanism [GO:0034739], histone H4K12 deacetylase activity, hydrolytic mechanism [GO:0140937], histone H4K5 deacetylase activity, hydrolytic mechanism [GO:0180032], histone H4K8 deacetylase activity, hydrolytic mechanism [GO:0180033], GO:1990162 Relationships: is_a histone deacetylase activity [GO:0004407]; is a type of GO:0016811 Note: Histone deacytylase (HDAC) enzymes are divided into four classes: the Class I Rpd3-like proteins (in human: HDAC1, HDAC2, HDAC3, and HDAC8); the Class II Hda1-like proteins (in human: HDAC4, HDAC5, HDAC6, HDAC7, HDAC9, and HDAC10); the Class III Sir2-like proteins (in human: SIRT1, SIRT2, SIRT3, SIRT4, SIRT5, SIRT6, and SIRT7); and the Class IV protein (HDAC11 in human). Except for Class III enzymes, the mechanism is a metal-dependent hydrolysis of the acetylated substrate. The Class III HDACs use NAD+ as a reactant to deacetylate acetyl lysine residues of protein substrates forming nicotinamide, the deacetylated product, and the metabolite 2'-O-acetyl-ADP-ribose. Therefore, Class III are classified as transferases (EC:2) and others are hydrolases (EC:3). References: PMID:24691964, PMID:28450737 Sources: RHEA:58196